vocalization behavior [GO:0071625] (biological process) Sources: GOC:mah Relationships: is a type of behavior [GO:0007610] Also known as: vocalisation behaviour Definition: The behavior in which an organism produces sounds by a mechanism involving its respiratory system. Subtypes: innate vocalization behavior [GO:0098582], learned vocalization behavior [GO:0098583]